{
  "gene_symbol": "HLA-F",
  "term_id": "GO:0001916",
  "gene_name": "HLA class I histocompatibility antigen, alpha chain F",
  "term_label": "positive regulation of T cell mediated cytotoxicity",
  "gene": "UniProtKB:P30511"
}